{
  "gene_name": "Monocarboxylate transporter 6",
  "gene_symbol": "SLC16A5",
  "gene": "UniProtKB:O15375",
  "term_label": "monocarboxylic acid transmembrane transporter activity",
  "term_id": "GO:0008028"
}